2-acylglycerophosphocholine O-acyltransferase activity [GO:0047190] (molecular function) Sources: RHEA:10332 Also known as: 2-acylglycerol-3-phosphorylcholine acyltransferase activity, 2-acylglycerophosphocholine acyltransferase activity, acyl-CoA:2-acyl-sn-glycero-3-phosphocholine O-acyltransferase activity Relationships: is a type of O-acyltransferase activity [GO:0008374] Definition: Catalysis of the reaction: 2-acyl-sn-glycero-3-phosphocholine + acyl-CoA = 1,2-diacyl-sn-glycero-3-phosphocholine + CoA.